germacrene A acid 8beta-hydroxylase activity [GO:0102614] (molecular function) Definition: Catalysis of the reaction: germacra-1(10),4,11(13)-trien-12-oate + O2 + reduced [NADPH--hemoprotein reductase] = 8beta-hydroxygermacra-1(10),4,11(13)-trien-12-oate + H(+) + H2O + oxidized [NADPH--hemoprotein reductase]. Sources: RHEA:57964 Relationships: is a type of GO:0016712